somatic portion of tanycyte [GO:1990017] (cellular component) Definition: Portion of a tanycyte that lies within the ependyma and contains the nucleus. A tanycyte is a specialized elongated ventricular ependymal cell that has processes that extend to the outer, or pial, surface of the CNS. Sources: ISBN:0195065719, NIF_Subcellular:sao401910342 Also known as: somatic portion Relationships: is a type of cell body [GO:0044297]